{
  "term_id": "GO:0016567",
  "gene_name": "Cullin-1",
  "gene": "UniProtKB:Q13616",
  "term_label": "protein ubiquitination",
  "gene_symbol": "CUL1"
}